{
  "gene_name": "Triadin",
  "term_id": "GO:0060047",
  "term_label": "heart contraction",
  "gene_symbol": "TRDN",
  "gene": "UniProtKB:Q13061"
}